{
  "gene": "UniProtKB:Q9H4H8",
  "gene_name": "Protein FAM83D",
  "term_id": "GO:0070372",
  "gene_symbol": "FAM83D",
  "term_label": "regulation of ERK1 and ERK2 cascade"
}